L-glucuronate reductase activity [GO:0047939] (molecular function) Also known as: glucuronate reductase activity, D-glucuronate reductase activity, D-glucuronate dehydrogenase activity, NADP-L-gulonate dehydrogenase activity, TPN-L-gulonate dehydrogenase activity, aldehyde reductase II activity, glucuronate dehydrogenase activity Relationships: is a type of oxidoreductase activity, acting on the CH-OH group of donors, NAD or NADP as acceptor [GO:0016616] Sources: EC:1.1.1.19, RHEA:14909 Definition: Catalysis of the reaction: L-gulonate + NADP+ = D-glucuronate + H+ + NADPH.